cyanidin 3-O-galactosyltransferase activity [GO:0102454] (molecular function) Relationships: is a type of hexosyltransferase activity [GO:0016758] Definition: Catalysis of the reaction: cyanidin + UDP-D-galactose = cyanidin 3-O-beta-D-galactoside betaine + UDP. Sources: RHEA:35631